{
  "gene_name": "Neurobeachin-like protein 2",
  "gene_symbol": "NBEAL2",
  "term_label": "platelet formation",
  "term_id": "GO:0030220",
  "gene": "UniProtKB:Q6ZNJ1"
}